{
  "term_id": "GO:0016514",
  "term_label": "SWI/SNF complex",
  "gene": "UniProtKB:Q92925",
  "gene_symbol": "SMARCD2",
  "gene_name": "SWI_SNF-related matrix-associated actin-dependent regulator of chromatin subfamily D member 2"
}